{
  "gene_name": "Cyclic nucleotide-gated cation channel beta-3",
  "term_id": "GO:0005222",
  "term_label": "intracellularly cAMP-activated cation channel activity",
  "gene": "UniProtKB:Q9NQW8",
  "gene_symbol": "CNGB3"
}